negative regulation of toll-like receptor 12 signaling pathway [GO:0034176] (biological process) Definition: Any process that stops, prevents, or reduces the frequency, rate, or extent of toll-like receptor 12 signaling pathway. References: PMID:16551253, PMID:17328678 Sources: GOC:add Also known as: negative regulation of TLR12 signaling pathway, negative regulation of toll-like receptor 12 signalling pathway Relationships: is a type of GO:0034175; is a type of GO:0039532; negatively regulates GO:0034174